DNA strand resection involved in replication fork processing [GO:0110025] (biological process) Definition: The 5' to 3' exonucleolytic resection of DNA at the site of a stalled replication fork that contributes to replication fork processing. References: PMID:28475874 Sources: GOC:mah Regulation: positively regulated by positive regulation of DNA strand resection involved in replication fork processing [GO:0106253]; regulated by regulation of DNA strand resection involved in replication fork processing [GO:0110026]; negatively regulated by negative regulation of DNA strand resection involved in replication fork processing [GO:0110027] Relationships: is a type of DNA metabolic process [GO:0006259]; is part of replication fork processing [GO:0031297]; has part GO:0035312